{
  "gene_symbol": "THG1L",
  "term_label": "Unknown cellular component",
  "gene": "UniProtKB:Q9NWX6",
  "gene_name": "Probable tRNA(His) guanylyltransferase",
  "term_id": "UNKNOWN:0003"
}